{
  "gene_name": "Complement receptor type 2",
  "gene": "UniProtKB:P20023",
  "gene_symbol": "CR2",
  "term_id": "GO:0002456",
  "term_label": "T cell mediated immunity"
}